phototransduction, visible light [GO:0007603] (biological process) Sources: GOC:go_curators, ISBN:0198506732 Definition: The sequence of reactions within a cell required to convert absorbed photons from visible light into a molecular signal. A visible light stimulus is electromagnetic radiation that can be perceived visually by an organism; for organisms lacking a visual system, this can be defined as light with a wavelength within the range 380 to 780 nm. Relationships: is a type of phototransduction [GO:0007602]; is a type of GO:0009584 Also known as: visual cascade, visual transduction